{
  "term_label": "phosphatidylinositol bisphosphate binding",
  "gene_symbol": "TTPAL",
  "term_id": "GO:1902936",
  "gene": "UniProtKB:Q9BTX7",
  "gene_name": "Alpha-tocopherol transfer protein-like"
}